{
  "gene_name": "Olfactory receptor 7G1",
  "gene": "UniProtKB:Q8NGA0",
  "gene_symbol": "OR7G1",
  "term_id": "GO:0007165",
  "term_label": "signal transduction"
}